TORC2 signaling [GO:0038203] (biological process) Sources: GOC:lb Regulation: regulated by regulation of TORC2 signaling [GO:1903939]; negatively regulated by GO:1903940; positively regulated by GO:1904515 Relationships: is_a TOR signaling [GO:0031929] Also known as: TORC2 signal transduction Definition: A series of intracellular molecular signals mediated by TORC2; TOR (rapamycin-insensitive companion of TOR) in complex with at least Rictor (regulatory-associated protein of TOR), or orthologs of, and other signaling components.